{
  "gene": "UniProtKB:O14807",
  "term_id": "GO:0007265",
  "gene_name": "Ras-related protein M-Ras",
  "term_label": "Ras protein signal transduction",
  "gene_symbol": "MRAS"
}